{
  "term_label": "trans-Golgi network",
  "gene_symbol": "TRAPPC9",
  "gene": "UniProtKB:Q96Q05",
  "term_id": "GO:0005802",
  "gene_name": "Trafficking protein particle complex subunit 9"
}